clavulanic acid biosynthetic process [GO:0033050] (BP) Also known as: clavulanic acid anabolism, clavulanic acid biosynthesis, clavulanic acid formation, clavulanic acid synthesis Sources: GOC:mah Definition: The chemical reactions and pathways resulting in the formation of clavulanic acid, (2R,3Z,5R)-3-(2-hydroxyethylidene)-7-oxo-4-oxa-1-azabicyclo[3.2.0]heptane-2-carboxylic acid. Relationships: is a type of GO:0072330; is a type of lactam biosynthetic process [GO:0072339]